DNA synthesis involved in DNA replication [GO:0090592] (biological process) Subtypes: GO:0019985, GO:0110166, DNA synthesis involved in mitotic DNA replication [GO:1904860] Sources: GOC:vw Definition: Synthesis of DNA that is a part of the process of duplicating one or more molecules of DNA. Relationships: is_a DNA biosynthetic process [GO:0071897]; is part of DNA replication [GO:0006260]